{
  "gene_name": "Insulin, isoform 2",
  "gene_symbol": "INS-IGF2",
  "term_label": "extracellular space",
  "term_id": "GO:0005615",
  "gene": "UniProtKB:F8WCM5"
}